positive regulation of cell size [GO:0045793] (biological process) Sources: GOC:go_curators Also known as: up regulation of cell size, up-regulation of cell size, upregulation of cell size, activation of cell size, stimulation of cell size Definition: Any process that increases cell size. Relationships: is a type of regulation of cell size [GO:0008361]